{
  "gene_symbol": "TMED7",
  "gene_name": "Transmembrane emp24 domain-containing protein 7",
  "gene": "UniProtKB:Q9Y3B3",
  "term_id": "GO:0006888",
  "term_label": "endoplasmic reticulum to Golgi vesicle-mediated transport"
}